deacetyl-[citrate-(pro-3S)-lyase] S-acetyltransferase activity [GO:0047187] (molecular function) Sources: EC:2.3.1.49, MetaCyc:2.3.1.49-RXN Definition: Catalysis of the reaction: deacetyl-[citrate-oxaloacetate-lyase ((pro-3S)-CH(2)COO(-)-acetate)] + S-acetylphosphopantetheine = [citrate oxaloacetate-lyase ((pro-3S)-CH(2)COO(-)-acetate)] + pantetheine 4'-phosphate. Relationships: is a type of GO:0016418; is a type of catalytic activity, acting on a protein [GO:0140096] Also known as: S-acetyl phosphopantetheine:deacetyl citrate lyase S-acetyltransferase activity, S-acetylphosphopantetheine:deacetyl-citrate-oxaloacetate-lyase((pro-3S)-CH2COO-rightacetate)S-acetyltransferase activity, deacetyl-citrate-(pro-3S)-lyase S-acetyltransferase activity, deacetyl-citrate-(pro-3S)-lyase acetyltransferase activity